{
  "gene_symbol": "ATG4B",
  "gene_name": "Cysteine protease ATG4B",
  "term_id": "GO:0000423",
  "term_label": "mitophagy",
  "gene": "UniProtKB:Q9Y4P1"
}